L-threonine 3-dehydrogenase activity [GO:0008743] (MF) Sources: EC:1.1.1.103, RHEA:13161 Definition: Catalysis of the reaction: L-threonine + NAD+ = L-2-amino-3-oxobutanoate + CO2 + NADH. Also known as: threonine 3-dehydrogenase activity, L-threonine dehydrogenase activity, L-threonine:NAD+ oxidoreductase activity, threonine dehydrogenase activity Relationships: is a type of oxidoreductase activity, acting on the CH-OH group of donors, NAD or NADP as acceptor [GO:0016616]